{
  "gene_symbol": "TSPY9",
  "term_label": "Unknown biological process",
  "gene_name": "Testis-specific Y-encoded protein 9",
  "gene": "UniProtKB:A0A494C1R9",
  "term_id": "UNKNOWN:0002"
}